{
  "term_id": "GO:0019901",
  "gene": "UniProtKB:P18031",
  "gene_symbol": "PTPN1",
  "term_label": "protein kinase binding",
  "gene_name": "Tyrosine-protein phosphatase non-receptor type 1"
}